{
  "gene_symbol": "CFAP58",
  "term_id": "GO:0005856",
  "gene_name": "Cilia- and flagella-associated protein 58",
  "gene": "UniProtKB:Q5T655",
  "term_label": "cytoskeleton"
}